nitrogen catabolite repression of transcription from RNA polymerase II promoter [GO:0001081] (biological process) Also known as: negative regulation of transcription from RNA polymerase II promoter by nitrogen catabolites Definition: A transcription regulation process in which the presence of one nitrogen source leads to a decrease in the frequency, rate, or extent of transcription, from an RNA polymerase II promoter, of specific genes involved in the metabolism of other nitrogen sources. Relationships: is a type of nitrogen catabolite regulation of transcription from RNA polymerase II promoter [GO:0001079]; is_a GO:0090295 References: PMID:19104072 Sources: GOC:mah, GOC:txnOH